{
  "term_id": "UNKNOWN:0002",
  "gene": "UniProtKB:Q8N9T2",
  "term_label": "Unknown biological process",
  "gene_name": "Putative uncharacterized protein CXorf42",
  "gene_symbol": "NKAPP1"
}